cilium [GO:0005929] (cellular component) Note: Note that we deem cilium and microtubule-based flagellum to be equivalent. In most eukaryotic species, intracellular sub-components of the cilium, such as the ciliary base and rootlet, are located near the plasma membrane. In Diplomonads such as Giardia, instead, the same ciliary parts are located further intracellularly. Also, 'cilium' may be used when axonemal structure and/or motility are unknown, or when axonemal structure is unusual. For all other cases, please refer to children of 'cilium'. Finally, note that any role of ciliary proteins in sensory events should be captured by annotating to relevant biological process terms. Relationships: is a type of membrane-bounded organelle [GO:0043227]; is a type of plasma membrane bounded cell projection [GO:0120025]; has part intraciliary transport particle [GO:0030990] Also known as: eukaryotic flagellum, microtubule-based flagellum, primary cilium, flagellum Subtypes: GO:0031514, non-motile cilium [GO:0097730] Definition: A specialized eukaryotic organelle that consists of a filiform extrusion of the cell surface and of some cytoplasmic parts. Each cilium is largely bounded by an extrusion of the cytoplasmic (plasma) membrane, and contains a regular longitudinal array of microtubules, anchored to a basal body. References: PMID:16824949, PMID:17009929, PMID:20144998 Sources: GOC:cilia, GOC:curators, GOC:kmv, GOC:vw, ISBN:0198547684